{
  "gene": "UniProtKB:O76094",
  "term_id": "GO:0005786",
  "gene_name": "Signal recognition particle subunit SRP72",
  "term_label": "signal recognition particle, endoplasmic reticulum targeting",
  "gene_symbol": "SRP72"
}